{
  "gene_name": "Anoctamin-10",
  "term_id": "GO:0005886",
  "term_label": "plasma membrane",
  "gene": "UniProtKB:Q9NW15",
  "gene_symbol": "ANO10"
}